{
  "gene_name": "Ribosomal oxygenase 2",
  "gene": "UniProtKB:Q8IUF8",
  "gene_symbol": "RIOX2",
  "term_id": "GO:0032453",
  "term_label": "histone H3K4 demethylase activity"
}